{
  "term_id": "GO:0005886",
  "gene": "UniProtKB:Q86UN2",
  "gene_name": "Reticulon-4 receptor-like 1",
  "term_label": "plasma membrane",
  "gene_symbol": "RTN4RL1"
}